{
  "gene_name": "Immunoglobulin lambda variable 3-19",
  "gene_symbol": "IGLV3-19",
  "term_label": "immune response",
  "term_id": "GO:0006955",
  "gene": "UniProtKB:P01714"
}